extrinsic component of intraperoxisomal membrane [GO:0005780] (cellular component) Sources: GOC:dos, GOC:jl, GOC:mah Also known as: extrinsic to intraperoxisomal membrane, intra-peroxisomal peripheral membrane Definition: The component of the intraperoxisomal membrane consisting of gene products and protein complexes that are loosely bound to one of its surfaces, but not integrated into the hydrophobic region. Relationships: is a type of GO:0031312; is part of peroxisomal membrane [GO:0005778]